inositol-3,4-bisphosphate 4-phosphatase activity [GO:0052828] (molecular function) Relationships: is_a inositol bisphosphate phosphatase activity [GO:0016312] Definition: Catalysis of the reaction: 1D-myo-inositol 3,4-bisphosphate + H2O = 1D-myo-inositol 3-phosphate + phosphate. Sources: GOC:mah